regulation of capsule organization [GO:1901913] (biological process) Also known as: regulation of capsule organisation, regulation of capsule organization and biogenesis Subtypes: regulation of capsule polysaccharide biosynthetic process [GO:0062084], negative regulation of capsule organization [GO:1901914], positive regulation of capsule organization [GO:1901915] Sources: GOC:TermGenie, GOC:di Definition: Any process that modulates the frequency, rate or extent of capsule organization. Relationships: is a type of regulation of cellular component organization [GO:0051128]; regulates capsule organization [GO:0045230]